{
  "gene_name": "Protein mab-21-like 3",
  "gene": "UniProtKB:Q8N8X9",
  "term_id": "UNKNOWN:0003",
  "term_label": "Unknown cellular component",
  "gene_symbol": "MAB21L3"
}